ferredoxin hydrogenase complex [GO:0009375] (cellular component) Definition: An enzyme complex that catalyzes the oxidation of reduced ferredoxin. Hydrogenase contains iron-sulfur clusters, and some contain nickel; it can use molecular hydrogen for the reduction of a variety of substances. Relationships: is a type of intracellular protein-containing complex [GO:0140535]; is a type of GO:1990204 References: PMID:12792025, PMID:9836629